viral genome circularization [GO:0099009] (BP) Relationships: is a type of viral process [GO:0016032] References: PMID:11894948, PMID:15489417, PMID:19523475, PMID:319596 Sources: VZ:3968 Definition: The circularization of a viral genome following infection of a host cell. This is common amongst bacterial viruses to protect the viral genome ends from nucleases, to convert the linear genome to an integrative precursor or to give rise to the replicative form of the genome. It can be mediated by covalent closure of the DNA sticky ends, recombinaison between redundant terminal sequences or via the binding of a protein at the viral DNA extremities.